{
  "gene_name": "T cell receptor alpha chain MC.7.G5",
  "term_label": "response to bacterium",
  "gene_symbol": "TRA",
  "term_id": "GO:0009617",
  "gene": "UniProtKB:P0DTU3"
}